{
  "gene_name": "Epidermal growth factor-like protein 6",
  "term_label": "Unknown molecular function",
  "gene_symbol": "EGFL6",
  "gene": "UniProtKB:Q8IUX8",
  "term_id": "UNKNOWN:0001"
}